3'-phosphoadenosine 5'-phosphosulfate transmembrane transporter activity [GO:0046964] (molecular function) Relationships: is a type of adenine nucleotide transmembrane transporter activity [GO:0000295]; is a type of purine ribonucleotide transmembrane transporter activity [GO:0005346]; is a type of sulfur compound transmembrane transporter activity [GO:1901682]; is part of 3'-phospho-5'-adenylyl sulfate transmembrane transport [GO:1902559] Also known as: 3'-phosphoadenosine 5'-phosphosulphate transporter activity, PAPS transporter activity, adenosine 3'-phosphate 5'-phosphosulfate transmembrane transporter activity Sources: ISBN:0198506732 Definition: Enables the transfer of 3'-phosphoadenosine 5'-phosphosulfate, a naturally occurring mixed anhydride synthesized from adenosine 5'-phosphosulfate, from one side of a membrane to the other.